{
  "gene_name": "Putative uncharacterized protein LOC401522",
  "term_id": "UNKNOWN:0003",
  "term_label": "Unknown cellular component",
  "gene": "UniProtKB:Q5VSD8",
  "gene_symbol": "Q5VSD8"
}